mesonephric interstitial fibroblast development [GO:0061267] (BP) Also known as: mesonephros interstitial cell development Sources: GOC:mtg_kidney_jan10 Relationships: is a type of renal interstitial fibroblast development [GO:0072141]; is part of mesonephric interstitial fibroblast differentiation [GO:0061266] Definition: The process whose specific outcome is the progression of a mesonephric interstitial fibroblast over time, from its formation to the mature structure.